{
  "gene": "UniProtKB:O43896",
  "gene_symbol": "KIF1C",
  "term_id": "GO:0008574",
  "gene_name": "Kinesin-like protein KIF1C",
  "term_label": "plus-end-directed microtubule motor activity"
}